regulation of leaf senescence [GO:1900055] (biological process) Definition: Any process that modulates the frequency, rate or extent of leaf senescence. Relationships: is_a regulation of developmental process [GO:0050793]; regulates leaf senescence [GO:0010150] Sources: GOC:TermGenie Subtypes: negative regulation of leaf senescence [GO:1900056], positive regulation of leaf senescence [GO:1900057]